{
  "gene_name": "UTP--glucose-1-phosphate uridylyltransferase",
  "gene": "UniProtKB:Q16851",
  "term_label": "UDP-alpha-D-glucose metabolic process",
  "gene_symbol": "UGP2",
  "term_id": "GO:0006011"
}